{
  "gene_name": "Keratin-associated protein 12-3",
  "gene_symbol": "KRTAP12-3",
  "term_id": "UNKNOWN:0003",
  "term_label": "Unknown cellular component",
  "gene": "UniProtKB:P60328"
}